{
  "term_label": "cytosol",
  "gene_symbol": "SPAG1",
  "gene": "UniProtKB:Q07617",
  "term_id": "GO:0005829",
  "gene_name": "Sperm-associated antigen 1"
}